{
  "gene_symbol": "SPINK8",
  "term_label": "Unknown molecular function",
  "term_id": "UNKNOWN:0001",
  "gene": "UniProtKB:P0C7L1",
  "gene_name": "Serine protease inhibitor Kazal-type 8"
}